{
  "gene_name": "E3 ubiquitin-protein ligase MIB1",
  "gene_symbol": "MIB1",
  "term_label": "endocytosis",
  "gene": "UniProtKB:Q86YT6",
  "term_id": "GO:0006897"
}